{
  "gene": "UniProtKB:O43795",
  "gene_name": "Unconventional myosin-Ib",
  "term_id": "GO:0000146",
  "term_label": "microfilament motor activity",
  "gene_symbol": "MYO1B"
}